(R,R)-butanediol dehydrogenase activity [GO:0000721] (molecular function) Sources: EC:1.1.1.4 Definition: Catalysis of the reversible reaction: (R,R)-butane-2,3-diol + NAD+ = (R)-acetoin + NADH + H+. Relationships: is a type of GO:0016616 Also known as: (R)-2,3-butanediol dehydrogenase activity, (R)-diacetyl reductase activity, 1-amino-2-propanol dehydrogenase activity, 1-amino-2-propanol oxidoreductase activity, 2,3-butanediol dehydrogenase activity, D-(-)-butanediol dehydrogenase activity, D-1-amino-2-propanol dehydrogenase activity, D-1-amino-2-propanol:NAD(2) oxidoreductase activity, D-aminopropanol dehydrogenase activity, D-butanediol dehydrogenase activity, aminopropanol oxidoreductase activity, butylene glycol dehydrogenase activity, butyleneglycol dehydrogenase activity, diacetyl (acetoin) reductase activity